{
  "gene": "UniProtKB:Q8N5G0",
  "term_id": "GO:0005743",
  "gene_symbol": "SMIM20",
  "gene_name": "Small integral membrane protein 20",
  "term_label": "mitochondrial inner membrane"
}